regulation of cytokinesis [GO:0032465] (biological process) Definition: Any process that modulates the frequency, rate or extent of the division of the cytoplasm of a cell and its separation into two daughter cells. Sources: GOC:mah Subtypes: negative regulation of cytokinesis [GO:0032466], positive regulation of cytokinesis [GO:0032467], GO:1902412, regulation of FtsZ-dependent cytokinesis [GO:2000244] Relationships: is a type of regulation of cell cycle process [GO:0010564]; is a type of regulation of cell division [GO:0051302]; RO_0002211 cytokinesis [GO:0000910] Also known as: regulation of cell cycle cytokinesis